{
  "term_label": "positive regulation of T cell differentiation",
  "gene_name": "Interleukin-36 beta",
  "gene": "UniProtKB:Q9NZH7",
  "term_id": "GO:0045582",
  "gene_symbol": "IL36B"
}